positive regulation of nitric oxide-cGMP mediated signal transduction [GO:0141150] (biological process) Definition: Any process that increases the rate, frequency or extent of nitric oxide-cGMP mediated signal transduction. Relationships: is a type of positive regulation of nitric oxide mediated signal transduction [GO:0010750]; is_a regulation of nitric oxide-cGMP mediated signal transduction [GO:0141149]; positively regulates GO:0038060 References: PMID:14615391